{
  "gene_name": "Putative 3-phosphoinositide-dependent protein kinase 2",
  "gene": "UniProtKB:Q6A1A2",
  "term_id": "GO:0035556",
  "gene_symbol": "PDPK2P",
  "term_label": "intracellular signal transduction"
}